regulation of gastric motility [GO:1905333] (BP) Relationships: is a type of regulation of digestive system process [GO:0044058]; regulates gastric motility [GO:0035482] References: PMID:9924029 Sources: GOC:TermGenie, GOC:als, GO_REF:0000058 Definition: Any process that modulates the frequency, rate or extent of gastric motility. Subtypes: regulation of gastric emptying [GO:0120060]